exit of virus from host cell nucleus [GO:0039674] (biological process) Definition: The directed movement of the viral genome or a viral particle out of the host cell nucleus. Sources: VZ:2177 Subtypes: exit of virus from host cell nucleus through nuclear pore [GO:0039675], exit of virus from host cell nucleus via nuclear envelope disassembly [GO:0039677], GO:0046802 Relationships: is a type of viral process [GO:0016032]; is a type of exit from host cell [GO:0035891]